{
  "gene_symbol": "TRMT13",
  "gene_name": "tRNA:m(4)X modification enzyme TRM13 homolog",
  "term_label": "tRNA methylation",
  "term_id": "GO:0030488",
  "gene": "UniProtKB:Q9NUP7"
}